positive regulation of antimicrobial peptide secretion [GO:0002796] (BP) Subtypes: GO:0002799, positive regulation of antifungal peptide secretion [GO:0002802] Relationships: is a type of positive regulation of antimicrobial peptide production [GO:0002225]; is a type of positive regulation of peptide secretion [GO:0002793]; is a type of regulation of antimicrobial peptide secretion [GO:0002794]; positively regulates antimicrobial peptide secretion [GO:0002776] Also known as: up regulation of antimicrobial peptide secretion, up-regulation of antimicrobial peptide secretion, upregulation of antimicrobial peptide secretion, activation of antimicrobial peptide secretion, stimulation of antimicrobial peptide secretion Definition: Any process that activates or increases the frequency, rate, or extent of antimicrobial peptide secretion. Sources: GOC:add